{
  "term_label": "RNA polymerase II cis-regulatory region sequence-specific DNA binding",
  "term_id": "GO:0000978",
  "gene_symbol": "SRY",
  "gene": "UniProtKB:Q05066",
  "gene_name": "Sex-determining region Y protein"
}